{
  "gene_name": "Zinc finger protein 496",
  "term_id": "UNKNOWN:0003",
  "term_label": "Unknown cellular component",
  "gene": "UniProtKB:Q96IT1",
  "gene_symbol": "ZNF496"
}